{
  "term_label": "DNA-binding transcription activator activity, RNA polymerase II-specific",
  "gene_name": "Replication initiator 1",
  "gene_symbol": "REPIN1",
  "gene": "UniProtKB:Q9BWE0",
  "term_id": "GO:0001228"
}